{
  "term_label": "DNA binding",
  "gene": "UniProtKB:Q5QNW6",
  "gene_symbol": "H2BC18",
  "gene_name": "Histone H2B type 2-F",
  "term_id": "GO:0003677"
}